{
  "gene_symbol": "AK4P3",
  "term_label": "AMP metabolic process",
  "gene_name": "Adenylate kinase 4, mitochondrial",
  "gene": "UniProtKB:A0A8I5KW96",
  "term_id": "GO:0046033"
}